positive regulation of gastric emptying [GO:0120062] (biological process) Relationships: is a type of positive regulation of digestive system process [GO:0060456]; is a type of GO:0120060; positively regulates gastric emptying [GO:0035483] Definition: Any process that increases the frequency, rate or extent of any gastric emptying process, the process in which the liquid and liquid-suspended solid contents of the stomach exit through the pylorus into the duodenum. References: PMID:15890336 Sources: GOC:sl